astrocyte-dopaminergic neuron signaling [GO:0036520] (biological process) Also known as: astrocyte-dopaminergic neuron cell signaling, mesencephalic dopaminergic neuron-astrocyte crosstalk, midbrain dopaminergic neuron-astrocyte crosstalk, dopaminergic neuron-astrocyte crosstalk References: PMID:12794311, PMID:21752258 Sources: GOC:PARL, GOC:bf Definition: Cell-cell signaling that mediates the transfer of information from an astrocyte to a dopaminergic neuron. Relationships: is a type of glial cell-neuron signaling [GO:0150098]